positive regulation of glycogen biosynthetic process [GO:0045725] (biological process) Sources: GOC:go_curators Relationships: is a type of regulation of glycogen biosynthetic process [GO:0005979]; is a type of positive regulation of macromolecule biosynthetic process [GO:0010557]; is_a GO:0070875; RO_0002213 glycogen biosynthetic process [GO:0005978] Also known as: positive regulation of glycogen anabolism, positive regulation of glycogen biosynthesis, positive regulation of glycogen formation, positive regulation of glycogen synthesis, up regulation of glycogen biosynthetic process, up-regulation of glycogen biosynthetic process, upregulation of glycogen biosynthetic process, activation of glycogen biosynthetic process, stimulation of glycogen biosynthetic process Definition: Any process that activates or increases the frequency, rate or extent of the chemical reactions and pathways resulting in the formation of glycogen.